{
  "gene_symbol": "ZKSCAN3",
  "gene_name": "Zinc finger protein with KRAB and SCAN domains 3",
  "term_id": "UNKNOWN:0003",
  "gene": "UniProtKB:Q9BRR0",
  "term_label": "Unknown cellular component"
}